{
  "term_id": "GO:0060326",
  "gene": "UniProtKB:O00421",
  "gene_name": "C-C chemokine receptor-like 2",
  "term_label": "cell chemotaxis",
  "gene_symbol": "CCRL2"
}